{
  "gene_symbol": "INSR",
  "gene_name": "Insulin receptor",
  "term_id": "GO:0042593",
  "term_label": "glucose homeostasis",
  "gene": "UniProtKB:P06213"
}